{
  "gene": "UniProtKB:Q9GZZ7",
  "gene_name": "GDNF family receptor alpha-4",
  "term_id": "GO:0043235",
  "term_label": "receptor complex",
  "gene_symbol": "GFRA4"
}